SCF-YDR131C ubiquitin ligase complex [GO:0097671] (cellular component) Definition: An SCF ubiquitin ligase complex in which the F-box protein is YDR131C in S. cerevisiae. References: PMID:14747994 Sources: GOC:jd, GOC:vw Relationships: is a type of GO:0019005